{
  "term_label": "regulation of transcription by RNA polymerase II",
  "gene_symbol": "ZNF317",
  "gene": "UniProtKB:Q96PQ6",
  "term_id": "GO:0006357",
  "gene_name": "Zinc finger protein 317"
}